neuronal ribonucleoprotein granule [GO:0071598] (cellular component) Definition: A ribonucleoprotein complex that is found in the cytoplasm of axons and dendrites, and transports translationally silenced mRNAs to dendritic synapses, where they are released and translated in response to specific exogenous stimuli. Relationships: is a type of cytoplasmic ribonucleoprotein granule [GO:0036464]; is part of neuron projection cytoplasm [GO:0120111] Also known as: neuronal RNP granule, neuronal RNA granule References: PMID:19015237, PMID:20368989 Sources: GOC:BHF, GOC:go_curators, GOC:mah